{
  "gene_symbol": "Q8N1X5",
  "term_id": "UNKNOWN:0002",
  "gene": "UniProtKB:Q8N1X5",
  "term_label": "Unknown biological process",
  "gene_name": "Uncharacterized protein FLJ37310"
}